{
  "term_label": "RNA endonuclease activity",
  "gene": "UniProtKB:Q9Y2C4",
  "gene_name": "Nuclease EXOG, mitochondrial",
  "gene_symbol": "EXOG",
  "term_id": "GO:0004521"
}